renal capsule morphogenesis [GO:0072128] (biological process) Definition: The process in which the anatomical structures of the renal capsule are generated and organized. The renal capsule is the tough fibrous layer surrounding the kidney, covered in a thick layer of perinephric adipose tissue. It provides some protection from trauma and damage. During development, it comprises a single layer of flattened cells that lie just above the cortical stroma and the condensed mesenchyme of the nephrogenic zone. It is in this region that the early stages of nephron induction and formation of new generations ureteric bud branches occur, as the kidney expands. Sources: GOC:mtg_kidney_jan10 Relationships: is a type of GO:0048729; is part of renal capsule development [GO:0072127] Subtypes: mesonephric capsule morphogenesis [GO:0061286], metanephric capsule morphogenesis [GO:0072265]